{
  "gene_symbol": "FBXO31",
  "gene": "UniProtKB:Q5XUX0",
  "term_id": "UNKNOWN:0001",
  "gene_name": "F-box only protein 31",
  "term_label": "Unknown molecular function"
}